{
  "term_id": "GO:0007612",
  "gene_symbol": "NRXN2",
  "gene_name": "Neurexin-2",
  "gene": "UniProtKB:Q9P2S2",
  "term_label": "learning"
}